{
  "term_label": "cellular response to growth factor stimulus",
  "gene_symbol": "TGFBR2",
  "term_id": "GO:0071363",
  "gene": "UniProtKB:P37173",
  "gene_name": "TGF-beta receptor type-2"
}